territorial aggressive behavior [GO:0002124] (biological process) Sources: GOC:hjd Definition: Aggressive behavior performed in defence of a fixed area against intruders, typically conspecifics. Relationships: is a type of aggressive behavior [GO:0002118] Also known as: territorial aggression